{
  "gene": "UniProtKB:Q96H40",
  "gene_symbol": "ZNF486",
  "term_id": "UNKNOWN:0003",
  "term_label": "Unknown cellular component",
  "gene_name": "Zinc finger protein 486"
}